mitochondrial DNA replication [GO:0006264] (biological process) Relationships: is a type of DNA-templated DNA replication [GO:0006261]; is a type of GO:0032042 Also known as: mtDNA replication, replication of mitochondrial DNA, mitochondrial DNA synthesis, mtDNA synthesis Sources: GOC:ai Subtypes: kinetoplast DNA replication [GO:0140909] Regulation: regulated by regulation of mitochondrial DNA replication [GO:0090296]; positively regulated by positive regulation of mitochondrial DNA replication [GO:0090297]; negatively regulated by negative regulation of mitochondrial DNA replication [GO:0090298] Definition: The process in which new strands of DNA are synthesized in the mitochondrion.